{
  "term_label": "Unknown cellular component",
  "gene_name": "Kita-kyushu lung cancer antigen 1",
  "gene": "UniProtKB:Q5H943",
  "gene_symbol": "CT83",
  "term_id": "UNKNOWN:0003"
}